{
  "gene_name": "Ankyrin repeat domain-containing protein 13B",
  "term_label": "late endosome",
  "gene_symbol": "ANKRD13B",
  "term_id": "GO:0005770",
  "gene": "UniProtKB:Q86YJ7"
}